{
  "gene_name": "Cysteinyl leukotriene receptor 2",
  "gene": "UniProtKB:Q9NS75",
  "term_id": "GO:0005886",
  "term_label": "plasma membrane",
  "gene_symbol": "CYSLTR2"
}